{
  "gene_name": "Zinc finger protein 461",
  "term_label": "DNA-binding transcription factor activity, RNA polymerase II-specific",
  "term_id": "GO:0000981",
  "gene_symbol": "ZNF461",
  "gene": "UniProtKB:Q8TAF7"
}